{
  "gene_name": "Calcitonin gene-related peptide type 1 receptor",
  "gene_symbol": "CALCRL",
  "gene": "UniProtKB:Q16602",
  "term_label": "plasma membrane",
  "term_id": "GO:0005886"
}